{
  "gene": "UniProtKB:Q5VVX9",
  "gene_name": "Ubiquitin-conjugating enzyme E2 U",
  "gene_symbol": "UBE2U",
  "term_label": "proteasome-mediated ubiquitin-dependent protein catabolic process",
  "term_id": "GO:0043161"
}